{
  "gene": "UniProtKB:Q9UI17",
  "gene_symbol": "DMGDH",
  "gene_name": "Dimethylglycine dehydrogenase, mitochondrial",
  "term_id": "GO:0005737",
  "term_label": "cytoplasm"
}